{
  "term_label": "nucleus",
  "term_id": "GO:0005634",
  "gene_symbol": "H2AL3",
  "gene": "UniProtKB:A0A3B3IU63",
  "gene_name": "Histone H2A-like 3"
}